{
  "term_id": "UNKNOWN:0002",
  "gene_symbol": "SUGCT",
  "term_label": "Unknown biological process",
  "gene": "UniProtKB:Q9HAC7",
  "gene_name": "Succinate--hydroxymethylglutarate CoA-transferase"
}